growth cone membrane [GO:0032584] (cellular component) Relationships: is a type of cellular anatomical structure [GO:0110165]; is part of plasma membrane [GO:0005886]; is part of GO:0030426 Definition: The portion of the plasma membrane surrounding a growth cone. Sources: GOC:mah